{
  "gene_name": "Leukocyte immunoglobulin-like receptor subfamily B member 2",
  "term_label": "immune response-inhibiting cell surface receptor signaling pathway",
  "gene": "UniProtKB:Q8N423",
  "gene_symbol": "LILRB2",
  "term_id": "GO:0002767"
}